regulation of turning behavior involved in mating [GO:0061094] (biological process) Relationships: is a type of regulation of male mating behavior [GO:1902435]; regulates turning behavior involved in mating [GO:0034607] Subtypes: positive regulation of turning behavior involved in mating [GO:0061095], negative regulation of turning behavior involved in mating [GO:0061096] Definition: Any process that modulates the rate, frequency or extent of turning behavior involved in mating. Turning behavior is the sharp ventral turn performed by the male as he approaches either the hermaphrodite head or tail, whilst trying to locate his partner's vulva. Turning occurs via a sharp ventral coil of the male's tail. Sources: GOC:dph, GOC:tb